cementum mineralization [GO:0071529] (BP) Also known as: cementum formation Relationships: is a type of GO:0034505 References: PMID:17043865 Sources: GOC:sl Definition: The process in which calcium salts, mainly carbonated hydroxyapatite, are deposited into the initial acellular cementum.